lateral pseudopodium assembly [GO:0031271] (biological process) Definition: The extension of a pseudopodium from the lateral area of a cell. Relationships: is a type of pseudopodium assembly [GO:0031269] Also known as: lateral pseudopodium formation Sources: GOC:dph, GOC:mah, GOC:pg, GOC:tb